microtubule nucleation by microtubule organizing center [GO:0051418] (biological process) Subtypes: astral microtubule nucleation [GO:0030954], microtubule nucleation by interphase microtubule organizing center [GO:0051415], microtubule nucleation by spindle pole body [GO:0051417], centrosome-templated microtubule nucleation [GO:0090222] Also known as: MTOC-mediated microtubule nucleation, microtubule nucleation by MTOC, microtubule nucleation by microtubule organising centre, microtubule organizing center-mediated microtubule nucleation Sources: GOC:ai Definition: The 'de novo' formation of a microtubule, mediated by the microtubule organizing center. Relationships: is a type of microtubule nucleation [GO:0007020]